primary leaflet morphogenesis [GO:0060778] (biological process) Definition: The process in which the primary leaflet attains its shape. A primary leaflet is a leaflet that develops directly from the rachis. Sources: GOC:dph, GOC:sdb_2009, GOC:tb Relationships: is a type of leaflet morphogenesis [GO:0060794]